{
  "term_label": "immune response",
  "gene_symbol": "IGKV1-37",
  "gene": "UniProtKB:A0A075B6S9",
  "term_id": "GO:0006955",
  "gene_name": "Probable non-functional immunoglobulinn kappa variable 1-37"
}